{
  "gene": "UniProtKB:Q13554",
  "term_label": "calcium/calmodulin-dependent protein kinase activity",
  "term_id": "GO:0004683",
  "gene_symbol": "CAMK2B",
  "gene_name": "Calcium_calmodulin-dependent protein kinase type II subunit beta"
}